Entner-Doudoroff pathway through gluconate to D-glyceraldehyde-3-phosphate [GO:0061681] (biological process) Definition: The Entner-Doudoroff pathway that proceeds through a D-gluconate intermediate and yields pyruvate and D-glyceraldehyde-3-phosphate. Relationships: is a type of glyceraldehyde-3-phosphate metabolic process [GO:0019682]; is_a Entner-Doudoroff pathway through gluconate [GO:0061679]; has part 2-dehydro-3-deoxygluconokinase activity [GO:0008673]; BFO_0000051 2-dehydro-3-deoxy-phosphogluconate aldolase activity [GO:0008675] References: PMID:12921536 Sources: GOC:dph